{
  "term_label": "Unknown biological process",
  "gene": "UniProtKB:Q9N2J8",
  "gene_symbol": "Q9N2J8",
  "gene_name": "HERV-H_2q24.1 provirus ancestral Env polyprotein",
  "term_id": "UNKNOWN:0002"
}